lipoteichoic acid biosynthetic process [GO:0070395] (biological process) Relationships: is a type of GO:0019350 Also known as: LTA biosynthetic process, lipoteichoic acid anabolism, lipoteichoic acid biosynthesis, lipoteichoic acid formation, lipoteichoic acid synthesis Definition: The chemical reactions and pathways resulting in the formation of lipoteichoic acid, which is a major component of the cell wall of gram-positive bacteria and typically consists of a chain of glycerol-phosphate repeating units linked to a glycolipid anchor. References: PMID:14665680, PMID:16020688 Sources: GOC:add